{
  "gene_name": "Probable G-protein coupled receptor 146",
  "term_id": "UNKNOWN:0002",
  "gene_symbol": "GPR146",
  "term_label": "Unknown biological process",
  "gene": "UniProtKB:Q96CH1"
}